MAP kinase kinase activity [GO:0004708] (molecular function) References: PMID:12623839, PMID:38270553 Subtypes: JUN kinase kinase activity [GO:0008545] Definition: Catalysis of the concomitant phosphorylation of threonine (T) and tyrosine (Y) residues in a T-X-Y motif in the activation loop of a MAP kinase (MAPK) substrate. Also known as: MEK activity, ERK activator kinase activity, MAPK activator activity, MAPKK activity, MAP kinase kinase 4 activity, MAP kinase kinase 7 activity, ATP:protein phosphotransferase (MAPKKK-activated) activity, MAP kinase or ERK kinase activity, MAP2K, MAPKK, MAPKK1, MEK1, MEK2, MKK, MKK2, MKK4, MKK6, MKK7, STK27, mitogen-activated protein kinase kinase activity Relationships: is a type of GO:0004712; is part of MAPK cascade [GO:0000165]